{
  "gene": "UniProtKB:P42566",
  "gene_symbol": "EPS15",
  "term_id": "GO:0006897",
  "term_label": "endocytosis",
  "gene_name": "Epidermal growth factor receptor substrate 15"
}